silver ion transport [GO:0015673] (biological process) Subtypes: silver ion transmembrane transport [GO:1902601] Also known as: silver transport Relationships: is a type of transition metal ion transport [GO:0000041] Definition: The directed movement of silver (Ag+) ions into, out of or within a cell, or between cells, by means of some agent such as a transporter or pore. Sources: GOC:ai